{
  "gene": "UniProtKB:O75128",
  "gene_name": "Protein cordon-bleu",
  "term_label": "perinuclear region of cytoplasm",
  "gene_symbol": "COBL",
  "term_id": "GO:0048471"
}